{
  "term_label": "Unknown cellular component",
  "gene": "UniProtKB:A8MV57",
  "term_id": "UNKNOWN:0003",
  "gene_symbol": "MPTX1",
  "gene_name": "Putative mucosal pentraxin homolog"
}